{
  "term_label": "extracellular space",
  "gene": "UniProtKB:Q9UBH0",
  "gene_name": "Interleukin-36 receptor antagonist protein",
  "gene_symbol": "IL36RN",
  "term_id": "GO:0005615"
}